nervous system process involved in regulation of systemic arterial blood pressure [GO:0001976] (biological process) Also known as: blood pressure regulation by neurological process, neurological process involved in regulation of systemic arterial blood pressure, neurological system process involved in regulation of systemic arterial blood pressure, fast control of arterial pressure Definition: The regulation of blood pressure mediated by detection of stimuli and a neurological response. Relationships: is a type of nervous system process [GO:0050877]; is part of GO:0003073 Subtypes: regulation of systemic arterial blood pressure by carotid sinus baroreceptor feedback [GO:0001978], regulation of systemic arterial blood pressure by chemoreceptor signaling [GO:0001979], GO:0001980, excitation of vasomotor center by chemoreceptor signaling [GO:0002008], excitation of vasomotor center by baroreceptor signaling [GO:0002010], brain renin-angiotensin system [GO:0002035], central nervous system control of baroreceptor feedback [GO:0003019], regulation of systemic arterial blood pressure by baroreceptor feedback [GO:0003025], regulation of systemic arterial blood pressure by aortic arch baroreceptor feedback [GO:0003026], circadian regulation of systemic arterial blood pressure by the suprachiasmatic nucleus [GO:0003054], GO:0003070 Sources: GOC:mtg_cardio, ISBN:0721643949